{
  "gene": "UniProtKB:A0A0A0MT96",
  "term_label": "Unknown molecular function",
  "term_id": "UNKNOWN:0001",
  "gene_symbol": "IGKJ3",
  "gene_name": "Immunoglobulin kappa joining 3 (Fragment)"
}